{
  "gene_name": "Mediator of RNA polymerase II transcription subunit 18",
  "term_label": "transcription coregulator activity",
  "gene": "UniProtKB:Q9BUE0",
  "gene_symbol": "MED18",
  "term_id": "GO:0003712"
}